{
  "term_id": "GO:0006955",
  "term_label": "immune response",
  "gene_symbol": "CCR9",
  "gene_name": "C-C chemokine receptor type 9",
  "gene": "UniProtKB:P51686"
}